peptidyl-proline dioxygenase activity [GO:0031543] (molecular function) Relationships: is a type of GO:0016706; is a type of GO:0140096 Also known as: proline hydroxylase activity, proline,2-oxoglutarate 4-dioxygenase activity, prolyl 4-hydroxylase activity, prolyl hydroxylase activity Definition: Catalysis of the reaction: peptidyl L-proline + 2-oxoglutarate + O2 = peptidyl hydroxy-L-proline + succinate + CO2. References: PMID:24550447, PMID:24550462 Sources: GOC:mah, GOC:vw Subtypes: procollagen-proline dioxygenase activity [GO:0019798], peptidyl-proline 3-dioxygenase activity [GO:0031544], peptidyl-proline 4-dioxygenase activity [GO:0031545]